{
  "gene_symbol": "RELA",
  "term_id": "GO:0005737",
  "gene": "UniProtKB:Q04206",
  "term_label": "cytoplasm",
  "gene_name": "Transcription factor p65"
}